tetrahydrodictyopterin binding [GO:0071576] (molecular function) Relationships: is a type of tetrahydrobiopterin binding [GO:0034617] Sources: GOC:mah, GOC:vw Definition: Binding to tetrahydrodictyopterin, the pterin 2-amino-6-[(1R,2R)-1,2-dihydroxypropyl]-5,6,7,8-tetrahydropteridin-4(3H)-one. Also known as: D-threo-tetrahydrobiopterin, DH4 binding